{
  "gene": "UniProtKB:Q9H1P6",
  "term_id": "UNKNOWN:0003",
  "gene_symbol": "C20orf85",
  "gene_name": "Uncharacterized protein C20orf85",
  "term_label": "Unknown cellular component"
}